{
  "term_id": "GO:0015746",
  "gene_name": "Sideroflexin-5",
  "term_label": "citrate transport",
  "gene_symbol": "SFXN5",
  "gene": "UniProtKB:Q8TD22"
}